distal portion of axoneme [GO:0120135] (cellular component) Sources: GOC:krc Relationships: is a type of cellular anatomical structure [GO:0110165]; is part of axoneme [GO:0005930] Definition: The portion of the axoneme that is close to the tip of the cilium. Also known as: distal part of axoneme